antifungal peptide secretion [GO:0002782] (biological process) Regulation: regulated by regulation of antifungal peptide secretion [GO:0002800]; RO_0002212 by negative regulation of antifungal peptide secretion [GO:0002801]; positively regulated by positive regulation of antifungal peptide secretion [GO:0002802] Relationships: is a type of GO:0002776; is part of antifungal peptide production [GO:0002781] References: PMID:11807545, PMID:15638771 Sources: GOC:add, ISBN:0781735149 Definition: The regulated release of an antifungal peptide from a cell or a tissue.